{
  "gene": "UniProtKB:Q5DT21",
  "term_id": "UNKNOWN:0003",
  "gene_name": "Serine protease inhibitor Kazal-type 9",
  "gene_symbol": "SPINK9",
  "term_label": "Unknown cellular component"
}